positive regulation of natural killer cell chemotaxis [GO:2000503] (biological process) Definition: Any process that activates or increases the frequency, rate or extent of natural killer cell chemotaxis. Sources: GOC:BHF Relationships: is a type of positive regulation of lymphocyte chemotaxis [GO:0140131]; is a type of regulation of natural killer cell chemotaxis [GO:2000501]; positively regulates natural killer cell chemotaxis [GO:0035747]